serotonin receptor complex [GO:0098665] (cellular component) Subtypes: serotonin-activated cation-selective channel complex [GO:1904602] Relationships: is a type of GO:0043235 Definition: A protein complex that is capable of serotonin receptor activity. Also known as: 5-HT receptor complex, 5-hydroxytryptamine receptor complex, 5HT receptor complex References: PMID:16116092 Sources: GOC:TermGenie, GOC:bhm, GO_REF:0000088